{
  "term_id": "UNKNOWN:0001",
  "gene_symbol": "C2orf42",
  "term_label": "Unknown molecular function",
  "gene_name": "Uncharacterized protein C2orf42",
  "gene": "UniProtKB:Q9NWW7"
}